{
  "gene": "UniProtKB:P62310",
  "gene_name": "U6 snRNA-associated Sm-like protein LSm3",
  "gene_symbol": "LSM3",
  "term_label": "P-body",
  "term_id": "GO:0000932"
}